{
  "gene_name": "Protein dispatched homolog 3",
  "gene_symbol": "DISP3",
  "gene": "UniProtKB:Q9P2K9",
  "term_id": "UNKNOWN:0002",
  "term_label": "Unknown biological process"
}